3'-flap-structured DNA binding [GO:0070337] (molecular function) Relationships: is a type of flap-structured DNA binding [GO:0070336] References: PMID:15189154 Sources: GOC:mah Definition: Binding to a 3'-flap structure in DNA. A DNA flap structure is one in which a single-stranded 3'-end of DNA or RNA protrudes from a double-stranded DNA molecule.